{
  "gene_name": "IgLON family member 5",
  "gene": "UniProtKB:A6NGN9",
  "gene_symbol": "IGLON5",
  "term_id": "GO:0007157",
  "term_label": "heterophilic cell-cell adhesion"
}